{
  "gene": "UniProtKB:Q6ZNG1",
  "gene_symbol": "ZNF600",
  "gene_name": "Zinc finger protein 600",
  "term_id": "GO:0000122",
  "term_label": "negative regulation of transcription by RNA polymerase II"
}